regulation of tooth mineralization [GO:0070170] (biological process) Definition: Any process that modulates the frequency, rate or extent of tooth mineralization, the deposition of calcium salts in tooth structures. Sources: GOC:BHF, GOC:mah Relationships: is a type of GO:0070167; regulates tooth mineralization [GO:0034505] Subtypes: negative regulation of tooth mineralization [GO:0070171], positive regulation of tooth mineralization [GO:0070172], GO:0070173